{
  "term_id": "UNKNOWN:0001",
  "gene": "UniProtKB:O60664",
  "term_label": "Unknown molecular function",
  "gene_name": "Perilipin-3",
  "gene_symbol": "PLIN3"
}